{
  "gene_symbol": "ANXA2",
  "gene_name": "Annexin A2",
  "gene": "UniProtKB:P07355",
  "term_id": "GO:0010756",
  "term_label": "positive regulation of plasminogen activation"
}